{
  "term_id": "GO:0005737",
  "gene_name": "ADP-ribosylation factor-like protein 17",
  "term_label": "cytoplasm",
  "gene_symbol": "ARL17A",
  "gene": "UniProtKB:Q8IVW1"
}